{
  "gene_name": "Transcription factor AP-2-alpha",
  "term_id": "GO:0001228",
  "term_label": "DNA-binding transcription activator activity, RNA polymerase II-specific",
  "gene": "UniProtKB:P05549",
  "gene_symbol": "TFAP2A"
}